{
  "gene": "UniProtKB:Q9UN37",
  "term_id": "GO:0043162",
  "gene_symbol": "VPS4A",
  "term_label": "ubiquitin-dependent protein catabolic process via the multivesicular body sorting pathway",
  "gene_name": "Vacuolar protein sorting-associated protein 4A"
}